{
  "gene": "UniProtKB:Q96P50",
  "term_id": "UNKNOWN:0001",
  "gene_symbol": "ACAP3",
  "gene_name": "Arf-GAP with coiled-coil, ANK repeat and PH domain-containing protein 3",
  "term_label": "Unknown molecular function"
}